{
  "gene": "UniProtKB:P48431",
  "term_label": "negative regulation of transcription by RNA polymerase II",
  "gene_symbol": "SOX2",
  "term_id": "GO:0000122",
  "gene_name": "Transcription factor SOX-2"
}